{
  "term_id": "GO:0042776",
  "term_label": "proton motive force-driven mitochondrial ATP synthesis",
  "gene_symbol": "ATP5PO",
  "gene": "UniProtKB:P48047",
  "gene_name": "ATP synthase subunit O, mitochondrial"
}